{
  "gene_symbol": "SMAD9",
  "gene_name": "Mothers against decapentaplegic homolog 9",
  "term_label": "transforming growth factor beta receptor signaling pathway",
  "term_id": "GO:0007179",
  "gene": "UniProtKB:O15198"
}